coated vesicle membrane [GO:0030662] (cellular component) Subtypes: ER to Golgi transport vesicle membrane [GO:0012507], COPI-coated vesicle membrane [GO:0030663], GO:0030665 Relationships: is a type of GO:0030659; is_a bounding membrane of organelle [GO:0098588]; is part of coated vesicle [GO:0030135] Definition: The lipid bilayer surrounding a coated vesicle. Sources: GOC:mah